atrial cardiac myofibril assembly [GO:0055004] (biological process) Also known as: atrial cardiac myofibril development, atrial heart myofibril development Sources: GOC:devbiol Relationships: is_a GO:0055003; is part of atrial cardiac muscle cell development [GO:0055014] Definition: The process whose specific outcome is the progression of the atrial cardiac myofibril over time, from its formation to the mature structure. A cardiac myofibril is a myofibril specific to cardiac muscle cells.